regulation of brassinosteroid biosynthetic process [GO:0010422] (biological process) Subtypes: GO:0010423, positive regulation of brassinosteroid biosynthetic process [GO:2000488] Definition: Any process that modulates the frequency, rate or extent of the chemical reactions and pathways resulting in the formation of brassinosteroids. References: PMID:16857903 Relationships: is a type of regulation of steroid hormone biosynthetic process [GO:0090030]; regulates brassinosteroid biosynthetic process [GO:0016132]